cellular response to selenite ion [GO:0072715] (biological process) Relationships: is a type of GO:0072714; is a type of GO:1901701 Sources: GOC:mah Definition: Any process that results in a change in state or activity of a cell (in terms of movement, secretion, enzyme production, gene expression, etc.) as a result of a selenite ion stimulus.